{
  "gene": "UniProtKB:Q9NPE6",
  "term_id": "GO:0043495",
  "gene_name": "Sperm-associated antigen 4 protein",
  "term_label": "protein-membrane adaptor activity",
  "gene_symbol": "SPAG4"
}